{
  "term_id": "GO:0019005",
  "term_label": "SCF ubiquitin ligase complex",
  "gene_name": "F-box only protein 4",
  "gene": "UniProtKB:Q9UKT5",
  "gene_symbol": "FBXO4"
}